positive regulation of the force of heart contraction by neuronal epinephrine-norepinephrine [GO:0003090] (biological process) Sources: GOC:mtg_cardio Also known as: increased force of heart contraction by epinephrine-norepinephrine released from the nerve endings, increased force of heart contraction by neuronal adrenaline-noradrenaline, increased force of heart contraction by neuronal epinephrine-norepinephrine, positive regulation of heart contraction by adrenaline-noradrenaline, positive regulation of heart contraction by epinephrine-norepinephrine Relationships: is a type of positive regulation of the force of heart contraction by epinephrine-norepinephrine [GO:0001997] Definition: Any process that increases the force with which the cardiac muscles of the heart pump blood through the circulatory system as a result of the presence of epinephrine or norepinephrine released from the nerve endings.